detection of chemical stimulus involved in sensory perception of sweet taste [GO:0001582] (BP) Definition: The series of events required for a sweet taste stimulus to be received and converted to a molecular signal. Sources: GOC:go_curators Also known as: perception of sweet taste, detection of chemical stimulus, perception of sweet taste, sensory transduction of chemical stimulus, sensory detection of chemical stimulus during perception of sweet taste, sensory detection of sweet taste, sensory transduction of chemical stimulus during perception of sweet taste, sensory transduction of sweet taste, sweet taste detection Relationships: is a type of detection of chemical stimulus involved in sensory perception of taste [GO:0050912]; BFO_0000050 sensory perception of sweet taste [GO:0050916]